C-C chemokine receptor activity [GO:0016493] (molecular function) Subtypes: C-C motif chemokine 19 receptor activity [GO:0038117], GO:0038121, GO:0038122, C-C motif chemokine 2 receptor activity [GO:0038149] Relationships: is a type of chemokine receptor activity [GO:0004950]; has part C-C chemokine binding [GO:0019957] Definition: Combining with a C-C chemokine and transmitting the signal from one side of the membrane to the other to initiate a change in cell activity. C-C chemokines do not have an amino acid between the first two cysteines of the characteristic four-cysteine motif. References: PMID:8662823 Sources: GOC:signaling